{
  "term_label": "voltage-gated potassium channel complex",
  "gene_symbol": "KCNIP4",
  "gene": "UniProtKB:Q6PIL6",
  "gene_name": "Kv channel-interacting protein 4",
  "term_id": "GO:0008076"
}